{
  "gene": "UniProtKB:Q15084",
  "term_label": "response to endoplasmic reticulum stress",
  "gene_symbol": "PDIA6",
  "gene_name": "Protein disulfide-isomerase A6",
  "term_id": "GO:0034976"
}